polyhydroxyalkanoate granule [GO:0070088] (cellular component) Definition: An inclusion body located in the cytoplasm of prokaryotes that consists of polyhydroxyalkanoate (PHA) molecules and associated proteins, surrounded by a phospholipid monolayer; the proteins include PHA synthase, PHA depolymerase and 3HB-oligomer hydroxylase, phasins (PhaPs), which are thought to be the major structural proteins of the membrane surrounding the inclusion, and the regulator of phasin expression PhaR. References: PMID:15762612 Sources: GOC:mah Also known as: carbonosome, PHA granule, PHB granule Relationships: is a type of inclusion body [GO:0016234]; is a type of GO:0043231; BFO_0000050 cytoplasm [GO:0005737]